{
  "term_label": "Unknown molecular function",
  "gene": "UniProtKB:Q9ULT8",
  "gene_name": "E3 ubiquitin-protein ligase HECTD1",
  "gene_symbol": "HECTD1",
  "term_id": "UNKNOWN:0001"
}